{
  "gene_symbol": "CTXN2",
  "gene": "UniProtKB:P0C2S0",
  "gene_name": "Cortexin-2",
  "term_label": "Unknown biological process",
  "term_id": "UNKNOWN:0002"
}